{
  "gene_name": "THAP domain-containing protein 8",
  "term_label": "Unknown cellular component",
  "term_id": "UNKNOWN:0003",
  "gene": "UniProtKB:Q8NA92",
  "gene_symbol": "THAP8"
}